{
  "gene": "UniProtKB:O15342",
  "gene_name": "V-type proton ATPase subunit e 1",
  "term_id": "GO:0000220",
  "gene_symbol": "ATP6V0E1",
  "term_label": "vacuolar proton-transporting V-type ATPase, V0 domain"
}